thiamine biosynthetic process [GO:0009228] (biological process) Regulation: regulated by GO:0070623; negatively regulated by negative regulation of thiamine biosynthetic process [GO:0070624]; positively regulated by GO:0090180 Subtypes: thiamine salvage [GO:0036172] Relationships: is_a thiamine metabolic process [GO:0006772]; is a type of primary alcohol biosynthetic process [GO:0034309]; is a type of GO:0042724 Definition: The chemical reactions and pathways resulting in the formation of thiamine (vitamin B1), a water soluble vitamin present in fresh vegetables and meats, especially liver. Sources: GOC:jl, ISBN:0198506732 Also known as: thiamin anabolism, thiamin biosynthetic process, thiamine biosynthesis, thiamine formation, thiamine synthesis, vitamin B1 biosynthesis, vitamin B1 biosynthetic process